{
  "gene": "UniProtKB:P27482",
  "term_id": "GO:0097720",
  "gene_symbol": "CALML3",
  "gene_name": "Calmodulin-like protein 3",
  "term_label": "calcineurin-mediated signaling"
}